{
  "gene_symbol": "ELMOD1",
  "gene": "UniProtKB:Q8N336",
  "gene_name": "ELMO domain-containing protein 1",
  "term_id": "GO:0005929",
  "term_label": "cilium"
}